{
  "gene_name": "Ribosomal protein S6 kinase beta-1",
  "term_id": "GO:0004674",
  "term_label": "protein serine/threonine kinase activity",
  "gene_symbol": "RPS6KB1",
  "gene": "UniProtKB:P23443"
}